{
  "gene_name": "Enhancer of polycomb homolog 1",
  "term_label": "regulation of transcription by RNA polymerase II",
  "gene": "UniProtKB:Q9H2F5",
  "term_id": "GO:0006357",
  "gene_symbol": "EPC1"
}